zearalenone biosynthetic process [GO:0106150] (biological process) Definition: The chemical reactions and pathways resulting in the formation of zearalenone, a mycotoxin produced by several Fusarium species, is most commonly found as a contaminant in stored grain and has chronic estrogenic effects on mammals. Relationships: is a type of GO:0033068; is a type of GO:0043386; is a type of phenol-containing compound biosynthetic process [GO:0046189] References: PMID:16517624, PMID:20578001 Sources: GOC:ach